{
  "gene_name": "Pleiotrophin",
  "gene": "UniProtKB:P21246",
  "gene_symbol": "PTN",
  "term_id": "GO:0005576",
  "term_label": "extracellular region"
}